craniofacial suture closure [GO:0160048] (BP) References: PMID:33842480 Relationships: is_a bone morphogenesis [GO:0060349] Definition: The process of fusing together the edges of a craniofacial suture.